{
  "term_id": "GO:0000978",
  "gene_name": "Homeobox protein engrailed-1",
  "gene_symbol": "EN1",
  "gene": "UniProtKB:Q05925",
  "term_label": "RNA polymerase II cis-regulatory region sequence-specific DNA binding"
}